{
  "term_id": "UNKNOWN:0003",
  "gene_name": "Inactive serine protease 35",
  "term_label": "Unknown cellular component",
  "gene_symbol": "PRSS35",
  "gene": "UniProtKB:Q8N3Z0"
}